{
  "term_label": "sensory perception of smell",
  "gene_symbol": "OR8B2",
  "term_id": "GO:0007608",
  "gene": "UniProtKB:Q96RD0",
  "gene_name": "Olfactory receptor 8B2"
}